{
  "gene_symbol": "DYNC2H1",
  "term_label": "9+2 motile cilium",
  "gene_name": "Cytoplasmic dynein 2 heavy chain 1",
  "term_id": "GO:0097729",
  "gene": "UniProtKB:Q8NCM8"
}